{
  "gene_name": "Claudin-9",
  "gene_symbol": "CLDN9",
  "term_id": "GO:0070830",
  "gene": "UniProtKB:O95484",
  "term_label": "bicellular tight junction assembly"
}